innate immune response [GO:0045087] (biological process) Definition: Innate immune responses are defense responses mediated by germline encoded components that directly recognize components of potential pathogens. Sources: GOC:add, GOC:ebc, GOC:mtg_sensu, GO_REF:0000022 Also known as: innate immunity, nonspecific immune response Relationships: is a type of immune response [GO:0006955]; is_a defense response to symbiont [GO:0140546] Subtypes: complement activation, lectin pathway [GO:0001867], innate immune response in mucosa [GO:0002227], GO:0002228, complement activation, alternative pathway [GO:0006957], GO:0009616, plant-type hypersensitive response [GO:0009626], GO:0009682, melanization defense response [GO:0035006], hemolymph coagulation [GO:0042381], GO:0046597, antifungal innate immune response [GO:0061760], GO:0090644, innate immunity memory response [GO:0090714], antibacterial innate immune response [GO:0140367], antiviral innate immune response [GO:0140374], complement activation, GZMK pathway [GO:0160257] Regulation: regulated by regulation of innate immune response [GO:0045088]; positively regulated by positive regulation of innate immune response [GO:0045089]; RO_0002212 by negative regulation of innate immune response [GO:0045824]